{
  "term_label": "Unknown cellular component",
  "gene_name": "Interleukin-2 receptor subunit alpha",
  "gene_symbol": "IL2RA",
  "gene": "UniProtKB:P01589",
  "term_id": "UNKNOWN:0003"
}